{
  "term_label": "Unknown cellular component",
  "gene": "UniProtKB:Q13113",
  "gene_name": "PDZK1-interacting protein 1",
  "gene_symbol": "PDZK1IP1",
  "term_id": "UNKNOWN:0003"
}